{
  "term_id": "UNKNOWN:0001",
  "gene_name": "Optic atrophy 3 protein",
  "term_label": "Unknown molecular function",
  "gene_symbol": "OPA3",
  "gene": "UniProtKB:Q9H6K4"
}